{
  "term_id": "GO:0005634",
  "term_label": "nucleus",
  "gene": "UniProtKB:A0A1B0GVX0",
  "gene_name": "LITAF domain-containing protein",
  "gene_symbol": "LITAFD"
}